{
  "term_id": "GO:0005886",
  "gene": "UniProtKB:P62330",
  "term_label": "plasma membrane",
  "gene_name": "ADP-ribosylation factor 6",
  "gene_symbol": "ARF6"
}